{
  "gene_symbol": "DNM1L",
  "term_label": "mitochondrial fragmentation involved in apoptotic process",
  "gene": "UniProtKB:O00429",
  "term_id": "GO:0043653",
  "gene_name": "Dynamin-1-like protein"
}